{
  "term_id": "GO:0008270",
  "gene": "UniProtKB:P62875",
  "gene_name": "DNA-directed RNA polymerases I, II, and III subunit RPABC5",
  "gene_symbol": "POLR2L",
  "term_label": "zinc ion binding"
}